{
  "gene_name": "CUGBP Elav-like family member 4",
  "term_label": "nucleus",
  "gene_symbol": "CELF4",
  "term_id": "GO:0005634",
  "gene": "UniProtKB:Q9BZC1"
}